{
  "gene": "UniProtKB:Q9UJH8",
  "gene_symbol": "METRN",
  "gene_name": "Meteorin",
  "term_label": "positive regulation of axonogenesis",
  "term_id": "GO:0050772"
}